melanin-concentrating hormone receptor binding [GO:0031776] (molecular function) Sources: GOC:mah, GOC:nln Relationships: is a type of neuropeptide receptor binding [GO:0071855] Also known as: melanin-concentrating hormone receptor ligand Definition: Binding to a melanin-concentrating hormone receptor. Subtypes: type 1 melanin-concentrating hormone receptor binding [GO:0031777], type 2 melanin-concentrating hormone receptor binding [GO:0031778]